{
  "gene_symbol": "NEK3",
  "gene": "UniProtKB:P51956",
  "term_id": "UNKNOWN:0001",
  "gene_name": "Serine_threonine-protein kinase Nek3",
  "term_label": "Unknown molecular function"
}